{
  "term_id": "UNKNOWN:0003",
  "term_label": "Unknown cellular component",
  "gene": "UniProtKB:Q6ZST4",
  "gene_symbol": "LCNL1",
  "gene_name": "Lipocalin-like 1 protein"
}